glycol metabolic process [GO:0042844] (biological process) References: PMID:9851711 Subtypes: anaerobic glycerol catabolic process to propane-1,3-diol [GO:0019589], GO:0034077, glycol biosynthetic process [GO:0042845], GO:0042846, 6-sulfoquinovose(1-) catabolic process to 3-sulfopropanediol(1-) [GO:0061721] Relationships: is a type of diol metabolic process [GO:0034311] Also known as: dihydric alcohol metabolic process, dihydric alcohol metabolism, glycol metabolism Definition: The chemical reactions and pathways involving glycol, a diol in which the two hydroxy groups are on different carbon atoms, usually but not necessarily adjacent.